{
  "term_label": "peroxisome fission",
  "gene_symbol": "OPA1",
  "gene": "UniProtKB:O60313",
  "gene_name": "Dynamin-like 120 kDa protein, mitochondrial",
  "term_id": "GO:0016559"
}